{
  "term_id": "UNKNOWN:0003",
  "gene_name": "Terminal nucleotidyltransferase 5D",
  "gene": "UniProtKB:Q8NEK8",
  "gene_symbol": "TENT5D",
  "term_label": "Unknown cellular component"
}